CD4-positive, CD25-positive, alpha-beta regulatory T cell differentiation [GO:0002361] (biological process) Definition: The process in which a precursor cell type acquires the specialized features of a CD4-positive, CD25-positive, alpha-beta regulatory T cell. References: PMID:15207821 Sources: GOC:add Also known as: CD4-positive, CD25-positive, alpha-beta regulatory T lymphocyte differentiation, CD4-positive, CD25-positive, alpha-beta regulatory T-cell differentiation, CD4-positive, CD25-positive, alpha-beta regulatory T-lymphocyte differentiation, CD4-positive, CD25-positive, alpha-beta regulatory T cell development Note: Note that immunologists typically use the word 'development' to refer to cells of B or T cell lineages undergoing the process that GO describes as 'cell differentiation'. Relationships: is a type of CD4-positive, alpha-beta T cell differentiation [GO:0043367]; is a type of regulatory T cell differentiation [GO:0045066] Subtypes: CD4-positive, CD25-positive, alpha-beta regulatory T cell differentiation involved in immune response [GO:0002298] Regulation: regulated by regulation of CD4-positive, CD25-positive, alpha-beta regulatory T cell differentiation [GO:0032829]; negatively regulated by GO:0032830; positively regulated by positive regulation of CD4-positive, CD25-positive, alpha-beta regulatory T cell differentiation [GO:0032831]